acharan sulfate lyase activity [GO:0052809] (molecular function) Definition: Catalysis of the cleavage of a carbon-oxygen bond in acharan sulfate, a glycosaminoglycan with a uniformly repeating disaccharide structure of alpha-D-N-acetylglucosaminyl-2-O-sulfo-alpha-L-iduronic acid. Relationships: is a type of carbon-oxygen lyase activity, acting on polysaccharides [GO:0016837] References: PMID:19566715 Sources: GOC:mengo_curators